pole plasm mRNA localization [GO:0019094] (BP) Sources: GOC:ai Definition: Any process in which mRNA is transported to, or maintained in, the oocyte pole plasm. An example of this is found in Drosophila melanogaster. Also known as: pole granule RNA localization, establishment and maintenance of mRNA localization in pole plasm, establishment and maintenance of pole plasm mRNA localization, oocyte pole plasm mRNA localization, pole plasm mRNA localisation Relationships: is a type of pole plasm RNA localization [GO:0007316]; is a type of intracellular mRNA localization involved in anterior/posterior axis specification [GO:0060811] Subtypes: pole plasm oskar mRNA localization [GO:0045451]